{
  "term_label": "Golgi membrane",
  "gene_name": "UbiA prenyltransferase domain-containing protein 1",
  "term_id": "GO:0000139",
  "gene": "UniProtKB:Q9Y5Z9",
  "gene_symbol": "UBIAD1"
}